{
  "gene_name": "Actin-related protein 5",
  "gene_symbol": "ACTR5",
  "term_label": "chromatin remodeling",
  "gene": "UniProtKB:Q9H9F9",
  "term_id": "GO:0006338"
}